{
  "term_id": "GO:0061640",
  "gene_name": "Septin-12",
  "gene": "UniProtKB:Q8IYM1",
  "term_label": "cytoskeleton-dependent cytokinesis",
  "gene_symbol": "SEPTIN12"
}